{
  "gene_symbol": "THSD7A",
  "term_label": "actin cytoskeleton organization",
  "gene_name": "Thrombospondin type-1 domain-containing protein 7A",
  "term_id": "GO:0030036",
  "gene": "UniProtKB:Q9UPZ6"
}